{
  "gene": "UniProtKB:P40933",
  "gene_name": "Interleukin-15",
  "term_label": "neutrophil activation",
  "term_id": "GO:0042119",
  "gene_symbol": "IL15"
}